carnitine biosynthetic process [GO:0045329] (biological process) Definition: The chemical reactions and pathways resulting in the formation of carnitine (hydroxy-trimethyl aminobutyric acid), a compound that participates in the transfer of acyl groups across the inner mitochondrial membrane. Sources: GOC:jl, ISBN:0198506732 Also known as: carnitine anabolism, carnitine biosynthesis, carnitine formation, carnitine synthesis, vitamin Bt biosynthesis, vitamin Bt biosynthetic process Relationships: is_a amino-acid betaine biosynthetic process [GO:0006578]; is a type of GO:0009437